{
  "term_id": "GO:0015171",
  "gene": "UniProtKB:Q8WY07",
  "gene_symbol": "SLC7A3",
  "gene_name": "Cationic amino acid transporter 3",
  "term_label": "amino acid transmembrane transporter activity"
}